{
  "gene_name": "Follicle-stimulating hormone receptor",
  "term_id": "GO:0008584",
  "gene_symbol": "FSHR",
  "term_label": "male gonad development",
  "gene": "UniProtKB:P23945"
}